{
  "gene_name": "Liprin-beta-1",
  "term_id": "GO:0007528",
  "gene_symbol": "PPFIBP1",
  "gene": "UniProtKB:Q86W92",
  "term_label": "neuromuscular junction development"
}